{
  "gene_symbol": "SLC1A3",
  "gene_name": "Excitatory amino acid transporter 1",
  "term_label": "L-glutamate transmembrane transporter activity",
  "gene": "UniProtKB:P43003",
  "term_id": "GO:0005313"
}